{
  "term_id": "GO:0030154",
  "gene": "UniProtKB:P41212",
  "gene_symbol": "ETV6",
  "term_label": "cell differentiation",
  "gene_name": "Transcription factor ETV6"
}